{
  "gene_name": "Zinc finger MYND domain-containing protein 10",
  "gene_symbol": "ZMYND10",
  "gene": "UniProtKB:O75800",
  "term_id": "GO:0044458",
  "term_label": "motile cilium assembly"
}